{
  "gene_name": "AP-1 complex subunit mu-2",
  "term_id": "GO:0005802",
  "term_label": "trans-Golgi network",
  "gene_symbol": "AP1M2",
  "gene": "UniProtKB:Q9Y6Q5"
}